{
  "gene_name": "Coiled-coil alpha-helical rod protein 1",
  "gene": "UniProtKB:Q8TD31",
  "term_label": "Unknown molecular function",
  "term_id": "UNKNOWN:0001",
  "gene_symbol": "CCHCR1"
}